regulation of interleukin-23 production [GO:0032667] (BP) Sources: GOC:mah Relationships: is a type of regulation of cytokine production [GO:0001817]; regulates interleukin-23 production [GO:0032627] Also known as: regulation of IL-23 biosynthetic process, regulation of IL-23 production, regulation of interleukin-23 anabolism, regulation of interleukin-23 biosynthesis, regulation of interleukin-23 biosynthetic process, regulation of interleukin-23 formation, regulation of interleukin-23 synthesis Subtypes: negative regulation of interleukin-23 production [GO:0032707], positive regulation of interleukin-23 production [GO:0032747] Definition: Any process that modulates the frequency, rate, or extent of interleukin-23 production.